{
  "term_id": "UNKNOWN:0001",
  "term_label": "Unknown molecular function",
  "gene": "UniProtKB:Q9UBI1",
  "gene_symbol": "COMMD3",
  "gene_name": "COMM domain-containing protein 3"
}